{
  "term_id": "GO:0043005",
  "gene": "UniProtKB:Q9GZP1",
  "term_label": "neuron projection",
  "gene_symbol": "NRSN2",
  "gene_name": "Neurensin-2"
}